{
  "term_id": "GO:1905323",
  "term_label": "telomerase holoenzyme complex assembly",
  "gene_symbol": "PTGES3",
  "gene": "UniProtKB:Q15185",
  "gene_name": "Prostaglandin E synthase 3"
}